{
  "gene_symbol": "DDR2",
  "term_id": "GO:0043235",
  "gene": "UniProtKB:Q16832",
  "term_label": "receptor complex",
  "gene_name": "Discoidin domain-containing receptor 2"
}